{
  "gene_symbol": "PTGES3",
  "term_label": "nucleus",
  "gene_name": "Prostaglandin E synthase 3",
  "gene": "UniProtKB:Q15185",
  "term_id": "GO:0005634"
}